{
  "term_id": "GO:0005886",
  "term_label": "plasma membrane",
  "gene_symbol": "EHBP1L1",
  "gene_name": "EH domain-binding protein 1-like protein 1",
  "gene": "UniProtKB:Q8N3D4"
}